cerebellar basket cell differentiation [GO:0021709] (biological process) References: PMID:15157725 Sources: GOC:cls, GOC:dgh, GOC:dph, GOC:jid, GO_REF:0000021 Relationships: is a type of cell differentiation in hindbrain [GO:0021533]; is a type of central nervous system neuron differentiation [GO:0021953]; is part of cerebellar molecular layer formation [GO:0021688] Definition: The process in which neuroblasts acquire specialized structural and/or functional features that characterize the mature cerebellar basket cell. Differentiation includes the processes involved in commitment of a neuroblast to a cerebellar basket cell fate. A cerebellar basket cell is an inhibitory GABAergic interneuron found in the cerebellar cortex.